{
  "gene_name": "Midnolin",
  "gene": "UniProtKB:Q504T8",
  "gene_symbol": "MIDN",
  "term_label": "Unknown molecular function",
  "term_id": "UNKNOWN:0001"
}